{
  "gene_symbol": "EIF3A",
  "term_id": "GO:0002188",
  "gene_name": "Eukaryotic translation initiation factor 3 subunit A",
  "gene": "UniProtKB:Q14152",
  "term_label": "translation reinitiation"
}